{
  "gene_name": "Protein phosphatase 1 regulatory inhibitor subunit 16B",
  "gene_symbol": "PPP1R16B",
  "gene": "UniProtKB:Q96T49",
  "term_id": "GO:0004857",
  "term_label": "enzyme inhibitor activity"
}